negative regulation of lymphoid progenitor cell differentiation [GO:1905457] (biological process) Relationships: is a type of GO:1901533; is_a regulation of lymphoid progenitor cell differentiation [GO:1905456]; negatively regulates lymphoid progenitor cell differentiation [GO:0002320] References: PMID:27010503 Sources: GOC:TermGenie, GO_REF:0000058 Also known as: down regulation of lymphoid progenitor cell differentiation, down-regulation of lymphoid progenitor cell differentiation, downregulation of lymphoid progenitor cell differentiation, inhibition of lymphoid progenitor cell differentiation Subtypes: negative regulation of pro-T cell differentiation [GO:2000175], negative regulation of pro-B cell differentiation [GO:2000974] Definition: Any process that stops, prevents or reduces the frequency, rate or extent of lymphoid progenitor cell differentiation.